oxidoreductase activity, acting on NAD(P)H, heme protein as acceptor [GO:0016653] (molecular function) Definition: Catalysis of an oxidation-reduction (redox) reaction in which NADH or NADPH acts as a hydrogen or electron donor and reduces a heme protein. Also known as: oxidoreductase activity, acting on NADH or NADPH, haem protein as acceptor, oxidoreductase activity, acting on NADH or NADPH, heme protein as acceptor Subtypes: GO:0003958, GO:0004128, leghemoglobin reductase [NAD(P)H] activity [GO:0015043], NADPH-cytochrome-c2 reductase activity [GO:0015047] Sources: GOC:ai Relationships: is a type of GO:0016651